{
  "term_label": "positive regulation of translational initiation",
  "term_id": "GO:0045948",
  "gene_name": "DNA-directed RNA polymerase II subunit RPB7",
  "gene_symbol": "POLR2G",
  "gene": "UniProtKB:P62487"
}